{
  "gene": "UniProtKB:Q63ZY3",
  "gene_symbol": "KANK2",
  "term_label": "cytoplasm",
  "gene_name": "KN motif and ankyrin repeat domain-containing protein 2",
  "term_id": "GO:0005737"
}